{
  "term_label": "forebrain development",
  "gene_symbol": "SOX2",
  "term_id": "GO:0030900",
  "gene_name": "Transcription factor SOX-2",
  "gene": "UniProtKB:P48431"
}